{
  "gene_symbol": "ACTN4",
  "gene_name": "Alpha-actinin-4",
  "term_label": "plasma membrane",
  "term_id": "GO:0005886",
  "gene": "UniProtKB:O43707"
}